{
  "gene_symbol": "ZNF479",
  "gene": "UniProtKB:Q96JC4",
  "term_label": "Unknown cellular component",
  "gene_name": "Zinc finger protein 479",
  "term_id": "UNKNOWN:0003"
}